{
  "gene_symbol": "XRCC2",
  "gene_name": "DNA repair protein XRCC2",
  "term_label": "double-strand break repair via homologous recombination",
  "term_id": "GO:0000724",
  "gene": "UniProtKB:O43543"
}